GABA receptor complex [GO:1902710] (cellular component) References: PMID:18790874 Sources: GOC:TermGenie, GOC:bhm, GO_REF:0000088 Subtypes: GABA-A receptor complex [GO:1902711], GO:1902712 Relationships: is a type of receptor complex [GO:0043235] Definition: A protein complex which is capable of GABA receptor activity. Upon binding of gamma-aminobutyric acid (GABA) it transmits the signal from one side of the membrane to the other to initiate a change in cell activity. Major inhibitory receptor in vertebrate brain. Also found in other vertebrate tissues, invertebrates and possibly in plants. Effective benzodiazepine receptor. Also known as: gamma-aminobutyric acid receptor complex